{
  "gene_symbol": "SLC41A2",
  "gene_name": "Solute carrier family 41 member 2",
  "term_id": "UNKNOWN:0002",
  "term_label": "Unknown biological process",
  "gene": "UniProtKB:Q96JW4"
}